{
  "term_label": "regulation of gene expression",
  "gene": "UniProtKB:A6NCK2",
  "gene_name": "Tripartite motif-containing protein 43B",
  "gene_symbol": "TRIM43B",
  "term_id": "GO:0010468"
}